DNA synthesis involved in UV-damage excision repair [GO:1904161] (biological process) Relationships: is_a DNA synthesis involved in DNA repair [GO:0000731]; is part of UV-damage excision repair [GO:0070914] Definition: Any DNA synthesis that is involved in UV-damage excision repair. References: PMID:10704216 Sources: GOC:TermGenie, GO_REF:0000060 Also known as: DNA synthesis involved in UV-damaged DNA endonuclease-dependent excision repair, DNA synthesis involved in UVDE-dependent excision repair, DNA synthesis involved in UVER, mitotic DNA repair synthesis involved in UV-damage excision repair, mitotic DNA repair synthesis involved in UV-damaged DNA endonuclease-dependent excision repair, mitotic DNA repair synthesis involved in UVDE-dependent excision repair, mitotic DNA repair synthesis involved in UVER, DNA synthesis during UV-damage excision repair, DNA synthesis during UV-damaged DNA endonuclease-dependent excision repair, DNA synthesis during UVDE-dependent excision repair, DNA synthesis during UVER, DNA synthesis involved in AER, DNA synthesis involved in alternative excision repair